{
  "term_id": "GO:0042392",
  "gene": "UniProtKB:Q8IY26",
  "gene_name": "Polyisoprenoid diphosphate_phosphate phosphohydrolase PLPP6",
  "term_label": "sphingosine-1-phosphate phosphatase activity",
  "gene_symbol": "PLPP6"
}